{
  "gene": "UniProtKB:O75865",
  "gene_symbol": "TRAPPC6A",
  "term_id": "GO:0006888",
  "term_label": "endoplasmic reticulum to Golgi vesicle-mediated transport",
  "gene_name": "Trafficking protein particle complex subunit 6A"
}